succinyl-CoA hydrolase activity [GO:0004778] (molecular function) Definition: Catalysis of the reaction: H2O + succinyl-CoA = CoA + H+ + succinate. Sources: EC:3.1.2.3, RHEA:11516 Also known as: succinyl coenzyme A deacylase activity, succinyl coenzyme A hydrolase activity, succinyl-CoA acylase activity Relationships: is a type of acyl-CoA hydrolase activity [GO:0016289]